{
  "gene_symbol": "FASTKD1",
  "term_label": "RNA binding",
  "gene_name": "FAST kinase domain-containing protein 1, mitochondrial",
  "gene": "UniProtKB:Q53R41",
  "term_id": "GO:0003723"
}